{
  "term_id": "GO:0007169",
  "gene_symbol": "EPHA1",
  "gene_name": "Ephrin type-A receptor 1",
  "term_label": "cell surface receptor protein tyrosine kinase signaling pathway",
  "gene": "UniProtKB:P21709"
}